positive regulation of ligase activity [GO:0051351] (biological process) Also known as: ligase activator, up regulation of ligase activity, up-regulation of ligase activity, upregulation of ligase activity, activation of ligase activity, stimulation of ligase activity Sources: GOC:ai Definition: Any process that activates or increases the frequency, rate or extent of ligase activity, the catalysis of the ligation of two substances with concomitant breaking of a diphosphate linkage, usually in a nucleoside triphosphate. Relationships: is_a positive regulation of catalytic activity [GO:0043085]; positively regulates ligase activity [GO:0016874] Subtypes: positive regulation of proton-transporting ATP synthase activity, rotational mechanism [GO:1905273]